{
  "gene_symbol": "MB21D2",
  "term_label": "Unknown cellular component",
  "gene_name": "Nucleotidyltransferase MB21D2",
  "term_id": "UNKNOWN:0003",
  "gene": "UniProtKB:Q8IYB1"
}